trigeminal ganglion development [GO:0061551] (biological process) Relationships: is a type of cranial ganglion development [GO:0061550] Also known as: trigeminal ganglia development Sources: GOC:dph Definition: The process whose specific outcome is the progression of a trigeminal ganglion over time, from its formation to the mature structure.